{
  "term_label": "cytoplasmic stress granule",
  "gene_name": "Ras GTPase-activating protein-binding protein 2",
  "gene": "UniProtKB:Q9UN86",
  "gene_symbol": "G3BP2",
  "term_id": "GO:0010494"
}